cyclohexanol oxidation [GO:0019399] (biological process) Definition: The cyclohexanol metabolic process in which cyclohexanol is converted to adipate. Sources: MetaCyc:CYCLOHEXANOL-OXIDATION-PWY Relationships: is a type of xenobiotic catabolic process [GO:0042178]